{
  "gene": "UniProtKB:O00471",
  "gene_name": "Exocyst complex component 5",
  "term_id": "GO:0006887",
  "gene_symbol": "EXOC5",
  "term_label": "exocytosis"
}